{
  "gene_symbol": "SNRPG",
  "term_label": "RNA binding",
  "gene": "UniProtKB:P62308",
  "term_id": "GO:0003723",
  "gene_name": "Small nuclear ribonucleoprotein G"
}